autophagy cargo adaptor activity [GO:0160247] (MF) Also known as: autophagy adaptor activity, selective autophagy receptor activity Relationships: is a type of protein-macromolecule adaptor activity [GO:0030674]; is part of substrate localization to autophagosome [GO:0061753] Definition: The binding activity of a molecule that brings together a cargo, targeted for degradation via autophagy, to a phagophore. References: PMID:23545414, PMID:31585693, PMID:36538890 Subtypes: autophagosome-membrane adaptor activity [GO:0160183]